turning behavior [GO:0035178] (biological process) Relationships: is a type of GO:0007626 References: PMID:10880478 Definition: Fine-tuning the spatial position of an organism in response to variability in their environment. For example, reorientation of an organism in the direction of a food source. Also known as: turning behaviour